sno(s)RNA 3'-end cleavage [GO:0043145] (biological process) Relationships: is a type of sno(s)RNA 3'-end processing [GO:0031126] References: PMID:12773397 Sources: GOC:go_curators Also known as: sno(s)RNA 3' end cleavage, sRNA 3'-end cleavage, snoRNA 3'-end cleavage Definition: The endonucleolytic cleavage of snoRNA 3' ends, which is required for mature snoRNAs to be functional.